{
  "gene_name": "Transmembrane 4 L6 family member 5",
  "gene_symbol": "TM4SF5",
  "term_id": "GO:0016020",
  "gene": "UniProtKB:O14894",
  "term_label": "membrane"
}